regulation of glutamate receptor signaling pathway [GO:1900449] (biological process) Definition: Any process that modulates the frequency, rate or extent of glutamate receptor signaling pathway. Relationships: is a type of regulation of signal transduction [GO:0009966]; regulates glutamate receptor signaling pathway [GO:0007215] Sources: GOC:BHF, GOC:TermGenie Subtypes: GO:0106426, negative regulation of glutamate receptor signaling pathway [GO:1900450], positive regulation of glutamate receptor signaling pathway [GO:1900451] Also known as: regulation of glutamate signaling pathway, regulation of glutamate signalling pathway